{
  "gene_symbol": "PTGER2",
  "term_label": "plasma membrane",
  "term_id": "GO:0005886",
  "gene": "UniProtKB:P43116",
  "gene_name": "Prostaglandin E2 receptor EP2 subtype"
}